{
  "term_label": "Set1C/COMPASS complex",
  "gene_symbol": "SETD1B",
  "gene_name": "Histone-lysine N-methyltransferase SETD1B",
  "term_id": "GO:0048188",
  "gene": "UniProtKB:Q9UPS6"
}